{
  "term_label": "Unknown cellular component",
  "gene_name": "FOXL2 neighbor protein",
  "gene": "UniProtKB:Q6ZUU3",
  "gene_symbol": "FOXL2NB",
  "term_id": "UNKNOWN:0003"
}